positive regulation of glutamine transport [GO:2000487] (biological process) Definition: Any process that activates or increases the frequency, rate or extent of glutamine transport. Sources: GOC:obol Also known as: positive regulation of L-glutamine transport Relationships: is a type of positive regulation of organic acid transport [GO:0032892]; is a type of GO:0051957; is a type of regulation of glutamine transport [GO:2000485]; positively regulates GO:0006868 Subtypes: positive regulation of L-glutamine import across plasma membrane [GO:1901036]